detection of chemical stimulus [GO:0009593] (biological process) Subtypes: detection of hypoxic conditions in blood by chemoreceptor signaling [GO:0002007], detection of unfolded protein [GO:0002235], GO:0002236, detection of hydrogen ion [GO:0003030], GO:0003031, GO:0003032, detection of calcium ion [GO:0005513], detection of nutrient [GO:0009594], detection of hormone stimulus [GO:0009720], detection of carbohydrate stimulus [GO:0009730], detection of salicylic acid stimulus [GO:0009752], GO:0009754, soluble molecule recognition [GO:0009995], detection of phosphate ion [GO:0010247], GO:0031319, detection of molecule of bacterial origin [GO:0032490], detection of molecule of fungal origin [GO:0032491], GO:0032492, detection of pheromone [GO:0043695], GO:0050907, GO:0051776 Definition: The series of events in which a chemical stimulus is received by a cell and converted into a molecular signal. Relationships: is a type of detection of stimulus [GO:0051606]; is part of GO:0042221 Also known as: chemoperception, detection of chemical substance, chemoreception, perception of chemical stimulus, perception of chemical substance Sources: GOC:jl